thiosulfate dehydrogenase activity [GO:0050338] (molecular function) Sources: EC:1.8.2.2, MetaCyc:THIOSULFATE-DEHYDROGENASE-RXN Also known as: thiosulphate dehydrogenase activity, tetrathionate synthase activity, thiosulfate oxidase activity, thiosulfate-acceptor oxidoreductase activity, thiosulfate-oxidizing enzyme, thiosulfate:ferricytochrome-c oxidoreductase activity Definition: Catalysis of the reaction: 2 thiosulfate + 2 ferricytochrome c = tetrathionate + 2 ferrocytochrome c. Relationships: is a type of GO:0016669